{
  "gene_name": "Importin subunit beta-1",
  "gene": "UniProtKB:Q14974",
  "gene_symbol": "KPNB1",
  "term_label": "cytoplasm",
  "term_id": "GO:0005737"
}